{
  "gene_symbol": "OR52L2P",
  "term_id": "UNKNOWN:0002",
  "gene_name": "Putative olfactory receptor 52L2",
  "gene": "UniProtKB:Q8NGH6",
  "term_label": "Unknown biological process"
}